{
  "term_label": "signaling receptor binding",
  "gene": "UniProtKB:Q8IU54",
  "term_id": "GO:0005102",
  "gene_symbol": "IFNL1",
  "gene_name": "Interferon lambda-1"
}